{
  "term_id": "GO:0005886",
  "term_label": "plasma membrane",
  "gene_name": "Tyrosine-protein kinase transmembrane receptor ROR2",
  "gene": "UniProtKB:Q01974",
  "gene_symbol": "ROR2"
}